{
  "term_label": "Unknown molecular function",
  "gene_name": "Neurensin-1",
  "gene_symbol": "NRSN1",
  "term_id": "UNKNOWN:0001",
  "gene": "UniProtKB:Q8IZ57"
}